{
  "term_label": "Unknown molecular function",
  "gene": "UniProtKB:A6NFY4",
  "term_id": "UNKNOWN:0001",
  "gene_symbol": "NEMP2",
  "gene_name": "Nuclear envelope integral membrane protein 2"
}